{
  "gene_name": "Kyphoscoliosis peptidase",
  "gene": "UniProtKB:Q8NBH2",
  "term_label": "muscle organ development",
  "term_id": "GO:0007517",
  "gene_symbol": "KY"
}